{
  "gene_symbol": "NRXN3",
  "gene": "UniProtKB:Q9Y4C0",
  "term_label": "plasma membrane",
  "term_id": "GO:0005886",
  "gene_name": "Neurexin-3"
}